{
  "gene_symbol": "GJE1",
  "gene_name": "Putative gap junction epsilon-1 protein",
  "term_label": "gap junction channel activity",
  "term_id": "GO:0005243",
  "gene": "UniProtKB:A6NN92"
}